{
  "gene_name": "Insulin growth factor-like family member 4",
  "term_id": "GO:0005615",
  "gene_symbol": "IGFL4",
  "term_label": "extracellular space",
  "gene": "UniProtKB:Q6B9Z1"
}